{
  "term_id": "GO:0005737",
  "gene_name": "Cytosolic carboxypeptidase 1",
  "gene": "UniProtKB:Q9UPW5",
  "term_label": "cytoplasm",
  "gene_symbol": "AGTPBP1"
}